regulation of cornification [GO:1905715] (biological process) Relationships: is a type of regulation of programmed cell death [GO:0043067]; regulates cornification [GO:0070268] Subtypes: negative regulation of cornification [GO:1905716], positive regulation of cornification [GO:1905717] Definition: Any process that modulates the frequency, rate or extent of cornification. References: PMID:26014679 Sources: GOC:TermGenie, GO_REF:0000058